positive regulation of protein exit from endoplasmic reticulum [GO:0070863] (biological process) Also known as: positive regulation of protein exit from ER, positive regulation of protein export from ER, positive regulation of protein export from endoplasmic reticulum, up regulation of protein exit from endoplasmic reticulum, up-regulation of protein exit from endoplasmic reticulum, upregulation of protein exit from endoplasmic reticulum, activation of protein exit from endoplasmic reticulum, stimulation of protein exit from endoplasmic reticulum Subtypes: positive regulation of retrograde protein transport, ER to cytosol [GO:1904154] Definition: Any process that activates or increases the frequency, rate or extent of directed movement of proteins from the endoplasmic reticulum. Relationships: is a type of regulation of protein exit from endoplasmic reticulum [GO:0070861]; is_a positive regulation of intracellular protein transport [GO:0090316]; positively regulates protein exit from endoplasmic reticulum [GO:0032527] Sources: GOC:mah